apoptotic process in response to mitochondrial fragmentation [GO:0140208] (biological process) References: PMID:18940801 Definition: Any apoptotic process that occurs as a result of mitochondrial fragmentation. Also known as: apoptosis in response to mitochondrial fragmentation Relationships: is a type of apoptotic process [GO:0006915]